{
  "gene": "UniProtKB:P41231",
  "gene_name": "P2Y purinoceptor 2",
  "term_label": "A1 adenosine receptor binding",
  "term_id": "GO:0031686",
  "gene_symbol": "P2RY2"
}